{
  "gene_name": "Centrosomal protein of 170 kDa protein B",
  "term_label": "Unknown cellular component",
  "gene": "UniProtKB:Q9Y4F5",
  "term_id": "UNKNOWN:0003",
  "gene_symbol": "CEP170B"
}